RS domain binding [GO:0050733] (molecular function) References: PMID:11684676, PMID:12215544 Definition: Binding to an RS domain of a protein; RS domains are usually highly phosphorylated and characterized by the presence of arginine (R)/serine (S) dipeptides. The RS domain promotes protein-protein interactions and directs subcellular localization and, in certain situations, nucleocytoplasmic shuttling of individual SR proteins. They also play a role in splicing. Relationships: is_a GO:0019904